{
  "term_label": "endoplasmic reticulum",
  "gene": "UniProtKB:Q13162",
  "gene_symbol": "PRDX4",
  "gene_name": "Peroxiredoxin-4",
  "term_id": "GO:0005783"
}